{
  "gene_name": "Immunoglobulin subtype domain-containing protein",
  "gene": "UniProtKB:A0A1W2PQM1",
  "term_id": "UNKNOWN:0001",
  "gene_symbol": "A0A1W2PQM1",
  "term_label": "Unknown molecular function"
}